{
  "term_id": "GO:0005634",
  "gene_symbol": "ZNF14",
  "gene": "UniProtKB:P17017",
  "term_label": "nucleus",
  "gene_name": "Zinc finger protein 14"
}